{
  "gene_symbol": "HTRA3",
  "term_label": "proteolysis",
  "gene": "UniProtKB:P83110",
  "term_id": "GO:0006508",
  "gene_name": "Serine protease HTRA3"
}